{
  "gene_symbol": "GAS7",
  "gene": "UniProtKB:O60861",
  "term_id": "GO:0030136",
  "gene_name": "Growth arrest-specific protein 7",
  "term_label": "clathrin-coated vesicle"
}